{
  "gene": "UniProtKB:Q99496",
  "gene_symbol": "RNF2",
  "gene_name": "E3 ubiquitin-protein ligase RING2",
  "term_id": "UNKNOWN:0002",
  "term_label": "Unknown biological process"
}